{
  "term_label": "positive regulation of mitochondrial fission",
  "gene_name": "Mitochondrial dynamics protein MIEF1",
  "gene": "UniProtKB:Q9NQG6",
  "term_id": "GO:0090141",
  "gene_symbol": "MIEF1"
}